regulation of synaptic vesicle cycle [GO:0098693] (biological process) Relationships: is_a regulation of vesicle-mediated transport [GO:0060627]; regulates GO:0099504 Subtypes: GO:0099162 Sources: GOC:dos Definition: Any process that modulates the frequency, rate or extent of the synaptic vesicle cycle.